{
  "gene": "UniProtKB:Q9BZX4",
  "gene_name": "Ropporin-1B",
  "term_label": "Unknown molecular function",
  "term_id": "UNKNOWN:0001",
  "gene_symbol": "ROPN1B"
}